{
  "gene": "UniProtKB:P22223",
  "term_id": "GO:0005737",
  "gene_name": "Cadherin-3",
  "term_label": "cytoplasm",
  "gene_symbol": "CDH3"
}